{
  "term_label": "neuron projection",
  "gene": "UniProtKB:P98160",
  "gene_name": "Basement membrane-specific heparan sulfate proteoglycan core protein",
  "gene_symbol": "HSPG2",
  "term_id": "GO:0043005"
}